{
  "term_id": "UNKNOWN:0002",
  "gene_symbol": "CT47B1",
  "term_label": "Unknown biological process",
  "gene_name": "Cancer_testis antigen family 47 member B1",
  "gene": "UniProtKB:P0C2W7"
}